{
  "gene": "UniProtKB:P55287",
  "term_label": "adherens junction organization",
  "term_id": "GO:0034332",
  "gene_name": "Cadherin-11",
  "gene_symbol": "CDH11"
}